{
  "term_label": "termination of RNA polymerase II transcription",
  "gene_name": "RNA polymerase II subunit A C-terminal domain phosphatase SSU72 like protein 2",
  "term_id": "GO:0006369",
  "gene": "UniProtKB:A0A1W2PQD8",
  "gene_symbol": "SSU72L2"
}